positive regulation of vitamin D biosynthetic process [GO:0060557] (biological process) Sources: CHEBI:27300, GOC:BHF, GOC:mah, ISBN:0471331309 Definition: Any process that increases the rate, frequency or extent of a vitamin D biosynthetic process. Vitamin D biosynthesis is the chemical reactions and pathways resulting in the formation of vitamin D, any of a group of related, fat-soluble compounds that are derived from delta-5,7 steroids and play a central role in calcium metabolism. Specific forms of vitamin D include calciferol (ergocalciferol; vitamin D2) and cholecalciferol (calciol; vitamin D3). Relationships: is_a positive regulation of steroid biosynthetic process [GO:0010893]; is a type of GO:0046136; is a type of regulation of vitamin D biosynthetic process [GO:0060556]; positively regulates vitamin D biosynthetic process [GO:0042368]